{
  "gene_name": "Superkiller complex protein 8",
  "term_label": "Unknown biological process",
  "gene": "UniProtKB:Q9GZS3",
  "term_id": "UNKNOWN:0002",
  "gene_symbol": "SKIC8"
}